{
  "term_label": "Unknown biological process",
  "gene_symbol": "DHRS13",
  "gene_name": "Dehydrogenase_reductase SDR family member 13",
  "gene": "UniProtKB:Q6UX07",
  "term_id": "UNKNOWN:0002"
}